{
  "term_label": "Unknown cellular component",
  "gene_symbol": "KNOP1",
  "gene": "UniProtKB:Q1ED39",
  "term_id": "UNKNOWN:0003",
  "gene_name": "Lysine-rich nucleolar protein 1"
}